{
  "term_id": "GO:0000030",
  "gene_name": "Probable C-mannosyltransferase DPY19L1",
  "gene_symbol": "DPY19L1",
  "term_label": "mannosyltransferase activity",
  "gene": "UniProtKB:Q2PZI1"
}